{
  "gene_name": "Zinc finger protein 333",
  "gene_symbol": "ZNF333",
  "gene": "UniProtKB:Q96JL9",
  "term_label": "regulation of transcription by RNA polymerase II",
  "term_id": "GO:0006357"
}